beta-1,4-mannosylglycolipid beta-1,3-N-acetylglucosaminyltransferase activity [GO:0046981] (molecular function) Also known as: UDP-N-acetylglucosamine:beta-D-mannosyl-glycolipid beta-1,3-N-acetylglucosaminyltransferase activity Definition: Catalysis of the transfer of N-acetylglucosamine (GlcNAc) in a beta-1,3 linkage to the mannose(beta-1,4)Glc disaccharide core of glycolipids. References: PMID:12130631, PMID:12130651 Sources: GOC:bf Relationships: is a type of acetylglucosaminyltransferase activity [GO:0008375]